{
  "term_label": "semaphorin receptor binding",
  "gene_symbol": "SEMA4B",
  "term_id": "GO:0030215",
  "gene": "UniProtKB:Q9NPR2",
  "gene_name": "Semaphorin-4B"
}